{
  "gene_name": "Pyrin",
  "term_id": "GO:0061630",
  "gene_symbol": "MEFV",
  "gene": "UniProtKB:O15553",
  "term_label": "ubiquitin protein ligase activity"
}